{
  "gene": "UniProtKB:Q494R0",
  "term_id": "UNKNOWN:0002",
  "gene_symbol": "FBXL19-AS1",
  "term_label": "Unknown biological process",
  "gene_name": "Putative uncharacterized protein FBXL19-AS1"
}